{
  "term_label": "RNA polymerase II cis-regulatory region sequence-specific DNA binding",
  "gene_name": "Homeobox protein Nkx-3.1",
  "gene": "UniProtKB:Q99801",
  "gene_symbol": "NKX3-1",
  "term_id": "GO:0000978"
}